thymus epithelium morphogenesis [GO:0097536] (biological process) Definition: The process in which the thymus epithelium is generated and organized. References: PMID:22342843 Sources: GOC:pr Also known as: thymic epithelium morphogenesis Relationships: is a type of morphogenesis of an epithelium [GO:0002009]; is part of thymus development [GO:0048538]